{
  "gene_name": "Testis-specific Y-encoded protein 3",
  "term_id": "GO:0000785",
  "gene_symbol": "TSPY3",
  "term_label": "chromatin",
  "gene": "UniProtKB:P0CV98"
}